lumenal side of cis-Golgi cisternae membrane [GO:0160277] (cellular component) Definition: The membrane leaflet of the cis-Golgi cisternae membrane that faces the Golgi lumen and is involved in glycosylation and lumen-facing cargo recognition. Also known as: lumenal face of cis-Golgi cisternae membrane, lumenal leaflet of cis-Golgi cisternae membrane References: PMID:23913272, PMID:34597626 Relationships: is a type of lumenal side of membrane [GO:0098576]; BFO_0000050 Golgi cis cisterna membrane [GO:1990674]